{
  "term_label": "synaptic membrane",
  "gene": "UniProtKB:Q6ZW31",
  "gene_name": "Rho GTPase-activating protein SYDE1",
  "gene_symbol": "SYDE1",
  "term_id": "GO:0097060"
}